cellular bud tip [GO:0005934] (cellular component) Definition: The end of a cellular bud distal to the site of attachment to the mother cell. Sources: GOC:mah Relationships: is a type of site of polarized growth [GO:0030427]; BFO_0000050 GO:0005933